{
  "gene_name": "Endothelin-1",
  "term_id": "GO:0045987",
  "term_label": "positive regulation of smooth muscle contraction",
  "gene": "UniProtKB:P05305",
  "gene_symbol": "EDN1"
}